metanephric glomerular mesangium development [GO:0072223] (biological process) Sources: GOC:mtg_kidney_jan10 Relationships: is a type of glomerular mesangium development [GO:0072109]; is part of metanephric glomerulus vasculature development [GO:0072239] Definition: The process whose specific outcome is the progression of the metanephric glomerular mesangium over time, from its formation to the mature structure. The metanephric glomerular mesangium is the thin membrane connective tissue composed of mesangial cells in the metanephros, which helps to support the capillary loops in a renal glomerulus.